{
  "gene_symbol": "BTBD1",
  "term_id": "GO:0022008",
  "gene_name": "BTB_POZ domain-containing protein 1",
  "term_label": "neurogenesis",
  "gene": "UniProtKB:Q9H0C5"
}